3,5 dichloro-THPH synthase activity [GO:0106267] (molecular function) References: PMID:20231486 Sources: RHEA:64360 Definition: Catalysis of the reaction: (3-chloro-2,4,6-trihydroxyphenyl)hexan-1-one + chloride + FADH2 + O2 = (3,5-dichloro-2,4,6-trihydroxyphenyl)hexan-1-one + FAD + 2 H2O. Relationships: is a type of oxidoreductase activity, acting on paired donors, with incorporation or reduction of molecular oxygen, reduced flavin or flavoprotein as one donor, and incorporation of one atom of oxygen [GO:0016712]